{
  "term_label": "Unknown molecular function",
  "term_id": "UNKNOWN:0001",
  "gene_name": "Tumor necrosis factor receptor superfamily member 6B",
  "gene_symbol": "TNFRSF6B",
  "gene": "UniProtKB:O95407"
}